{
  "gene": "UniProtKB:P29474",
  "gene_name": "Nitric oxide synthase 3",
  "term_id": "GO:0004517",
  "gene_symbol": "NOS3",
  "term_label": "nitric-oxide synthase activity"
}